{
  "gene_name": "Gametocyte-specific factor 1",
  "term_label": "Unknown molecular function",
  "term_id": "UNKNOWN:0001",
  "gene": "UniProtKB:Q8WW33",
  "gene_symbol": "GTSF1"
}